{
  "term_label": "detection of chemical stimulus involved in sensory perception of smell",
  "term_id": "GO:0050911",
  "gene_name": "Olfactory receptor 2M7",
  "gene": "UniProtKB:Q8NG81",
  "gene_symbol": "OR2M7"
}